{
  "gene_symbol": "FYCO1",
  "term_id": "GO:1901098",
  "gene_name": "FYVE and coiled-coil domain-containing protein 1",
  "term_label": "positive regulation of autophagosome maturation",
  "gene": "UniProtKB:Q9BQS8"
}